{
  "term_label": "female meiosis I",
  "gene": "UniProtKB:A2RUB1",
  "term_id": "GO:0007144",
  "gene_symbol": "MEIOC",
  "gene_name": "Meiosis-specific coiled-coil domain-containing protein MEIOC"
}